{
  "term_label": "B cell activation involved in immune response",
  "term_id": "GO:0002312",
  "gene_name": "Interferon alpha-16",
  "gene": "UniProtKB:P05015",
  "gene_symbol": "IFNA16"
}